{
  "term_id": "GO:0003810",
  "gene_symbol": "TGM6",
  "gene_name": "Protein-glutamine gamma-glutamyltransferase 6",
  "gene": "UniProtKB:O95932",
  "term_label": "protein-glutamine gamma-glutamyltransferase activity"
}